eurydendroid cell differentiation [GO:0021755] (biological process) Relationships: is a type of GO:0021533; is a type of central nervous system neuron differentiation [GO:0021953]; is part of cerebellar cortex formation [GO:0021697] Definition: The process in which neuroblasts acquire specialized structural and/or functional features that characterize the mature eurydendroid cell. Differentiation includes the processes involved in commitment of a neuroblast to a eurydendroid cell fate. A eurydendroid cell is an efferent neuron found in the cerebellar cortex of teleosts. References: PMID:15892096 Sources: GOC:cls, GOC:dgh, GOC:dph, GOC:jid, GO_REF:0000021